guanine nucleotide transport [GO:0001408] (BP) Definition: The directed movement of guanine nucleotides, GTP, GDP, and/or GMP, into, out of or within a cell, or between cells, by means of some agent such as a transporter or pore. Sources: GOC:mcc Relationships: is a type of GO:0015865 Subtypes: GO:0070731, guanine nucleotide transmembrane transport [GO:1903790]